{
  "gene": "UniProtKB:Q14031",
  "term_id": "GO:0038063",
  "gene_symbol": "COL4A6",
  "gene_name": "Collagen alpha-6(IV) chain",
  "term_label": "collagen-activated tyrosine kinase receptor signaling pathway"
}